{
  "term_label": "Unknown molecular function",
  "gene": "UniProtKB:Q3KRA6",
  "term_id": "UNKNOWN:0001",
  "gene_name": "UPF0538 protein C2orf76",
  "gene_symbol": "C2orf76"
}